{
  "gene": "UniProtKB:P20592",
  "term_id": "GO:0005874",
  "term_label": "microtubule",
  "gene_symbol": "MX2",
  "gene_name": "Interferon-induced GTP-binding protein Mx2"
}